threonyl-tRNA aminoacylation [GO:0006435] (biological process) Sources: GOC:mcc, ISBN:0716730510 Relationships: is a type of tRNA aminoacylation for protein translation [GO:0006418] Subtypes: GO:0070159 Definition: The process of coupling threonine to threonyl-tRNA, catalyzed by threonyl-tRNA synthetase. The threonyl-tRNA synthetase is a class-II synthetase. The activated amino acid is transferred to the 3'-OH group of a threonine-accetping tRNA.